{
  "term_id": "GO:0060271",
  "gene": "UniProtKB:Q96M11",
  "gene_name": "Centriolar and ciliogenesis-associated protein HYLS1",
  "term_label": "cilium assembly",
  "gene_symbol": "HYLS1"
}